{
  "term_label": "regulation of transcription by RNA polymerase II",
  "gene": "UniProtKB:Q6ZN18",
  "gene_symbol": "AEBP2",
  "term_id": "GO:0006357",
  "gene_name": "Zinc finger protein AEBP2"
}